{
  "term_id": "GO:0007165",
  "gene_symbol": "CTTN",
  "gene_name": "Src substrate cortactin",
  "gene": "UniProtKB:Q14247",
  "term_label": "signal transduction"
}